{
  "gene": "UniProtKB:Q9UBT2",
  "gene_name": "SUMO-activating enzyme subunit 2",
  "term_label": "cytoplasm",
  "term_id": "GO:0005737",
  "gene_symbol": "UBA2"
}